squalene monooxygenase activity [GO:0004506] (molecular function) Definition: Catalysis of the reaction: H+ + NADPH + O2 + squalene = (S)-2,3-epoxysqualene + H2O + NADP+. Sources: RHEA:25282 Also known as: squalene,NADPH:oxygen oxidoreductase (2,3-epoxidizing) activity, squalene 2,3-oxidocyclase activity, squalene epoxidase activity, squalene hydroxylase activity, squalene oxydocyclase activity, squalene-2,3-epoxidase activity, squalene-2,3-epoxide cyclase activity Relationships: is a type of oxidoreductase activity, acting on paired donors, with incorporation or reduction of molecular oxygen, NAD(P)H as one donor, and incorporation of one atom of oxygen [GO:0016709]